nucleocytoplasmic transport complex [GO:0031074] (CC) Sources: GOC:mah Also known as: nucleocytoplasmic shuttling complex Definition: Any complex that acts to move proteins or RNAs into or out of the nucleus through nuclear pores. Subtypes: GO:0042564, RNA nuclear export complex [GO:0042565] Relationships: is a type of GO:0032991